{
  "term_id": "UNKNOWN:0002",
  "gene_name": "Chromodomain Y-like protein 2",
  "gene": "UniProtKB:Q8N8U2",
  "term_label": "Unknown biological process",
  "gene_symbol": "CDYL2"
}